{
  "gene": "UniProtKB:Q8IZV2",
  "gene_name": "CKLF-like MARVEL transmembrane domain-containing protein 8",
  "gene_symbol": "CMTM8",
  "term_id": "GO:0019911",
  "term_label": "structural constituent of myelin sheath"
}